arabinan transmembrane transport [GO:0042899] (biological process) Relationships: is a type of polysaccharide transport [GO:0015774]; is a type of carbohydrate transmembrane transport [GO:0034219] Also known as: arabinan transport Definition: The process in which arabinan is transported across a lipid bilayer, from one side of a membrane to the other. Sources: GOC:jl